{
  "gene": "UniProtKB:Q9BQP9",
  "term_label": "Unknown cellular component",
  "gene_name": "BPI fold-containing family A member 3",
  "gene_symbol": "BPIFA3",
  "term_id": "UNKNOWN:0003"
}